13-series resolvin biosynthetic process [GO:0106298] (biological process) Definition: The chemical reactions and pathways resulting in the formation of resolvin family 13-series, hydroxy fatty acids derived from docosapentaenoic acid. Relationships: is a type of resolvin biosynthetic process [GO:0106295] References: PMID:26236990